{
  "term_label": "serotonin-gated monoatomic cation channel activity",
  "gene": "UniProtKB:Q9GZZ6",
  "term_id": "GO:0022850",
  "gene_name": "Neuronal acetylcholine receptor subunit alpha-10",
  "gene_symbol": "CHRNA10"
}